{
  "gene": "UniProtKB:Q2TAA5",
  "term_label": "dolichol-linked oligosaccharide biosynthetic process",
  "gene_name": "GDP-Man:Man(3)GlcNAc(2)-PP-Dol alpha-1,2-mannosyltransferase",
  "gene_symbol": "ALG11",
  "term_id": "GO:0006488"
}